{
  "term_label": "Unknown biological process",
  "term_id": "UNKNOWN:0002",
  "gene": "UniProtKB:P48307",
  "gene_name": "Tissue factor pathway inhibitor 2",
  "gene_symbol": "TFPI2"
}